{
  "term_label": "eosinophil chemotaxis",
  "gene_symbol": "CCL19",
  "gene_name": "C-C motif chemokine 19",
  "term_id": "GO:0048245",
  "gene": "UniProtKB:Q99731"
}